{
  "term_id": "GO:0005739",
  "term_label": "mitochondrion",
  "gene": "UniProtKB:Q93073",
  "gene_symbol": "SECISBP2L",
  "gene_name": "Selenocysteine insertion sequence-binding protein 2-like"
}